negative regulation of termination of DNA-templated transcription [GO:0060567] (biological process) Subtypes: GO:0031564, negative regulation of termination of RNA polymerase II transcription [GO:0120191], negative regulation of termination of RNA polymerase I transcription [GO:2000731] Relationships: is a type of GO:0031554; is a type of negative regulation of protein-containing complex disassembly [GO:0043242]; is a type of negative regulation of DNA-templated transcription [GO:0045892]; negatively regulates DNA-templated transcription termination [GO:0006353] Also known as: negative regulation of DNA-dependent transcription, termination, negative regulation of DNA-templated transcription, termination, negative regulation of termination of DNA-dependent transcription, negative regulation of transcription termination, DNA-dependent Sources: GOC:dph, GOC:tb, GOC:txnOH Definition: Any process that decreases the rate, frequency or extent of DNA-dependent transcription termination, the process in which transcription is completed; the formation of phosphodiester bonds ceases, the RNA-DNA hybrid dissociates, and RNA polymerase releases the DNA.